{
  "gene_name": "PDZ domain-containing protein MAGIX",
  "gene_symbol": "MAGIX",
  "term_label": "Unknown biological process",
  "term_id": "UNKNOWN:0002",
  "gene": "UniProtKB:Q9H6Y5"
}